{
  "term_id": "GO:0071294",
  "gene_symbol": "MT1G",
  "gene": "UniProtKB:P13640",
  "term_label": "cellular response to zinc ion",
  "gene_name": "Metallothionein-1G"
}